pancreas regeneration [GO:1990798] (biological process) Definition: The regrowth of a destroyed pancreas. Relationships: is a type of GO:0031100 References: PMID:1985964